export across cell outer membrane [GO:0140317] (BP) Definition: The directed movement of a substance across the outer membrane in cells with two membranes. Subtypes: xenobiotic detoxification by transmembrane export across the cell outer membrane [GO:0140330] Relationships: is a type of transmembrane transport [GO:0055085] References: PMID:15968039